{
  "term_label": "RNA polymerase II preinitiation complex assembly",
  "gene_symbol": "TAF6L",
  "term_id": "GO:0051123",
  "gene_name": "TAF6-like RNA polymerase II p300_CBP-associated factor-associated factor 65 kDa subunit 6L",
  "gene": "UniProtKB:Q9Y6J9"
}